{
  "term_id": "GO:1902711",
  "term_label": "GABA-A receptor complex",
  "gene_symbol": "GABRP",
  "gene": "UniProtKB:O00591",
  "gene_name": "Gamma-aminobutyric acid receptor subunit pi"
}